negative regulation of monocyte extravasation [GO:2000438] (biological process) Sources: GOC:obol Definition: Any process that stops, prevents or reduces the frequency, rate or extent of monocyte extravasation. Relationships: is a type of negative regulation of cellular extravasation [GO:0002692]; is a type of negative regulation of mononuclear cell migration [GO:0071676]; is a type of regulation of monocyte extravasation [GO:2000437]; negatively regulates monocyte extravasation [GO:0035696]